{
  "term_id": "GO:0005737",
  "gene": "UniProtKB:Q86Z20",
  "gene_symbol": "CCDC125",
  "term_label": "cytoplasm",
  "gene_name": "Coiled-coil domain-containing protein 125"
}